{
  "gene": "UniProtKB:O43581",
  "gene_name": "Synaptotagmin-7",
  "term_label": "vesicle-mediated transport",
  "term_id": "GO:0016192",
  "gene_symbol": "SYT7"
}